{
  "gene": "UniProtKB:Q96JQ0",
  "gene_symbol": "DCHS1",
  "gene_name": "Protocadherin-16",
  "term_label": "beta-catenin binding",
  "term_id": "GO:0008013"
}